positive regulation of xenophagy [GO:1904417] (biological process) Note: An example of this is mouse Tbk1 (UniProt symbol, Q9WUN2) in PMID:21617041 (inferred from mutant phenotype). Definition: Any process that activates or increases the frequency, rate or extent of xenophagy. Also known as: up regulation of xenophagy, up-regulation of xenophagy, upregulation of xenophagy, activation of xenophagy References: PMID:21617041 Sources: GOC:PARL, GOC:TermGenie, GOC:pad, GO_REF:0000058 Relationships: is a type of positive regulation of macroautophagy [GO:0016239]; is a type of positive regulation of defense response [GO:0031349]; is a type of GO:0032103; is a type of regulation of xenophagy [GO:1904415]; positively regulates xenophagy [GO:0098792]